{
  "gene_name": "Olfactory receptor 13A1",
  "gene": "UniProtKB:Q8NGR1",
  "term_id": "UNKNOWN:0002",
  "gene_symbol": "OR13A1",
  "term_label": "Unknown biological process"
}